{
  "gene_name": "PI-PLC X domain-containing protein 2",
  "term_label": "phosphoric diester hydrolase activity",
  "gene": "UniProtKB:Q0VAA5",
  "term_id": "GO:0008081",
  "gene_symbol": "PLCXD2"
}